L-arginine catabolic process [GO:0006527] (biological process) Definition: The chemical reactions and pathways resulting in the breakdown of L-arginine, 2-amino-5-(carbamimidamido)pentanoic acid. Sources: GOC:go_curators Relationships: is a type of GO:0006525; is a type of glutamine family amino acid metabolic process [GO:0009064]; is_a L-amino acid catabolic process [GO:0170035]; is a type of proteinogenic amino acid catabolic process [GO:0170040] Also known as: arginine breakdown, arginine catabolism, arginine degradation Regulation: regulated by GO:1900081; negatively regulated by negative regulation of arginine catabolic process [GO:1900082] Subtypes: L-arginine catabolic process to L-proline [GO:0019493], L-arginine catabolic process to L-glutamate [GO:0019544], L-arginine catabolic process to succinate [GO:0019545], L-arginine deiminase pathway [GO:0019546]